methionine-tRNA ligase activity [GO:0004825] (MF) Relationships: is a type of aminoacyl-tRNA ligase activity [GO:0004812] Definition: Catalysis of the reaction: ATP + L-methionine + tRNA(Met) = AMP + diphosphate + L-methionyl-tRNA(Met). Also known as: methionyl-tRNA synthetase activity, L-methionine:tRNAMet ligase (AMP-forming), MetRS activity, methionine translase activity, methionyl-transfer RNA synthetase activity, methionyl-transfer ribonucleate synthetase activity, methionyl-transfer ribonucleic acid synthetase activity Sources: EC:6.1.1.10